regulation of heptadecane biosynthetic process [GO:1900896] (biological process) Definition: Any process that modulates the frequency, rate or extent of heptadecane biosynthetic process. Sources: GOC:TermGenie, GOC:mengo_curators Also known as: regulation of heptadecane anabolism, regulation of heptadecane biosynthesis, regulation of heptadecane formation, regulation of heptadecane synthesis Relationships: is a type of regulation of alkane biosynthetic process [GO:1901577]; regulates GO:1900636 Subtypes: negative regulation of heptadecane biosynthetic process [GO:1900897], positive regulation of heptadecane biosynthetic process [GO:1900898]